L-tyrosine import across plasma membrane [GO:1903808] (BP) Also known as: L-tyrosine import, L-tyrosine import into cell, L-tyrosine uptake Regulation: regulated by GO:1900929; negatively regulated by negative regulation of L-tyrosine import across plasma membrane [GO:1900930]; positively regulated by positive regulation of L-tyrosine import across plasma membrane [GO:1900931] Relationships: is a type of tyrosine transport [GO:0015828]; is a type of amino acid import across plasma membrane [GO:0089718]; is a type of L-alpha-amino acid transmembrane transport [GO:1902475] References: PMID:23895341 Sources: GOC:TermGenie, GO_REF:0000075 Definition: The directed movement of L-tyrosine from outside of a cell, across the plasma membrane and into the cytosol.